{
  "gene_name": "Potassium voltage-gated channel subfamily A member 1",
  "term_label": "synapse",
  "gene_symbol": "KCNA1",
  "gene": "UniProtKB:Q09470",
  "term_id": "GO:0045202"
}